{
  "gene_name": "E3 ubiquitin-protein ligase RNF166",
  "gene_symbol": "RNF166",
  "term_label": "Unknown cellular component",
  "gene": "UniProtKB:Q96A37",
  "term_id": "UNKNOWN:0003"
}